{
  "gene_name": "Protein FAM50B",
  "gene": "UniProtKB:Q9Y247",
  "term_label": "Unknown molecular function",
  "gene_symbol": "FAM50B",
  "term_id": "UNKNOWN:0001"
}